anthocyanidin 3-O-glucosyltransferase activity [GO:0047213] (molecular function) Relationships: is a type of GO:0035251 Sources: EC:2.4.1.115, MetaCyc:2.4.1.115-RXN Also known as: 3-GT activity, UDP-D-glucose:anthocyanidin 3-O-beta-D-glucosyltransferase activity, UDP-glucose:anthocyanidin 3-O-D-glucosyltransferase activity, UDP-glucose:anthocyanidin/flavonol 3-O-glucosyltransferase activity, UDP-glucose:cyanidin-3-O-glucosyltransferase activity, uridine diphosphoglucose-anthocyanidin 3-O-glucosyltransferase activity Definition: Catalysis of the reaction: anthocyanidin + UDP-D-glucose = anthocyanidin-3-O-D-glucoside + UDP.